{
  "gene": "UniProtKB:P51858",
  "gene_name": "Hepatoma-derived growth factor",
  "term_id": "GO:0006338",
  "term_label": "chromatin remodeling",
  "gene_symbol": "HDGF"
}